{
  "term_label": "endopolyphosphatase activity",
  "gene": "UniProtKB:Q96G61",
  "gene_symbol": "NUDT11",
  "gene_name": "Diphosphoinositol polyphosphate phosphohydrolase 3-beta",
  "term_id": "GO:0000298"
}